meiotic mismatch repair [GO:0000710] (biological process) Definition: A system for the identification and correction of base-base mismatches, small insertion-deletion loops, and regions of heterology that are present in duplex DNA formed with strands from two recombining molecules. Correction of the mismatch can result in non-Mendelian segregation of alleles following meiosis. References: PMID:10357855 Sources: GOC:elh Relationships: is a type of mismatch repair [GO:0006298]; is a type of meiosis I cell cycle process [GO:0061982] Subtypes: GO:0010776, GO:0010777